cell-cell junction organization [GO:0045216] (BP) Sources: GOC:ai, GOC:dph, GOC:jl, GOC:mah Subtypes: desmosome organization [GO:0002934], cell-cell junction assembly [GO:0007043], plasmodesma organization [GO:0009663], adherens junction organization [GO:0034332], cell-cell junction maintenance [GO:0045217], GO:0120193, cell-cell junction disassembly [GO:0150147] Relationships: is a type of GO:0034330 Also known as: cell-cell junction assembly and maintenance, cell-cell junction organisation, intercellular junction assembly and maintenance, cell-cell junction biogenesis Definition: A process that is carried out at the cellular level which results in the assembly, arrangement of constituent parts, or disassembly of a cell-cell junction. A cell-cell junction is a specialized region of connection between two cells.